{
  "gene_name": "Receptor activity-modifying protein 2",
  "term_label": "receptor internalization",
  "term_id": "GO:0031623",
  "gene": "UniProtKB:O60895",
  "gene_symbol": "RAMP2"
}